mitochondrial prolyl-tRNA aminoacylation [GO:0070157] (biological process) Relationships: is a type of prolyl-tRNA aminoacylation [GO:0006433]; is a type of GO:0070127 Definition: The process of coupling proline to prolyl-tRNA in a mitochondrion, catalyzed by prolyl-tRNA synthetase. In tRNA aminoacylation, the amino acid is first activated by linkage to AMP and then transferred to either the 2'- or the 3'-hydroxyl group of the 3'-adenosine residue of the tRNA. Sources: GOC:mah, GOC:mcc